host cell mitochondrial inner membrane [GO:0044192] (CC) Definition: The inner, i.e. lumen-facing, lipid bilayer of the host cell mitochondrial envelope. It is highly folded to form cristae. Relationships: is a type of host cell mitochondrial membrane [GO:0044191] Sources: GOC:jl